{
  "gene_name": "Barttin",
  "gene": "UniProtKB:Q8WZ55",
  "term_label": "chloride transport",
  "term_id": "GO:0006821",
  "gene_symbol": "BSND"
}